ERBB4-EGFR signaling pathway [GO:0038137] (biological process) Definition: The series of molecular signals transmitted by a heterodimeric complex of the tyrosine kinase receptors EGFR (epidermal growth factor receptor/ERBB1) and ERBB4. The pathway begins with binding of a ligand to either cell surface receptor, or the dimeric receptor complex, and ends with regulation of a downstream cellular process, e.g. transcription. References: PMID:16460914 Sources: GOC:signaling Relationships: is_a epidermal growth factor receptor signaling pathway [GO:0007173]; is a type of GO:0038130 Also known as: ERBB1-ERBB4 signaling pathway, ERBB4-EGFR signalling pathway, HER1-HER4 signaling pathway